{
  "gene": "UniProtKB:Q99490",
  "term_id": "GO:0016020",
  "gene_name": "Arf-GAP with GTPase, ANK repeat and PH domain-containing protein 2",
  "term_label": "membrane",
  "gene_symbol": "AGAP2"
}